{
  "term_id": "GO:0030141",
  "gene_symbol": "KLK6",
  "gene_name": "Kallikrein-6",
  "term_label": "secretory granule",
  "gene": "UniProtKB:Q92876"
}